{
  "gene_name": "CREB-binding protein",
  "gene": "UniProtKB:Q92793",
  "gene_symbol": "CREBBP",
  "term_id": "GO:0000123",
  "term_label": "histone acetyltransferase complex"
}